negative regulation of dendritic spine morphogenesis [GO:0061002] (biological process) Definition: Any process that decreases the rate, frequency, or extent of dendritic spine morphogenesis, the process in which the anatomical structures of a dendritic spine are generated and organized. A dendritic spine is a protrusion from a dendrite and a specialized subcellular compartment involved in synaptic transmission. Relationships: is a type of negative regulation of neuron projection development [GO:0010977]; is a type of negative regulation of dendritic spine development [GO:0061000]; is a type of regulation of dendritic spine morphogenesis [GO:0061001]; negatively regulates dendritic spine morphogenesis [GO:0060997] Sources: GOC:dph